endoplasmic reticulum polarization [GO:0061163] (biological process) Relationships: is a type of GO:0007029 Also known as: ER polarization, ER localization involved in ER polarization at cell division site, endoplasmic reticulum localisation involved in endoplasmic reticulum polarization at cell division site, endoplasmic reticulum localization involved in endoplasmic reticulum polarization at cell division site, establishment of endoplasmic reticulum localisation involved in endoplasmic reticulum polarization at cell division site, establishment of endoplasmic reticulum localization involved in endoplasmic reticulum polarization at cell division site, maintenance of endoplasmic reticulum location involved in endoplasmic reticulum polarization at cell division site, transitional endoplasmic reticulum polarization at cell division site Sources: GOC:dph, GOC:vw Definition: The endoplasmic reticulum organization process that results in the structure of the endoplasmic reticulum being oriented in the cell. Endoplasmic reticulum polarization serves as a mechanism to compartmentalize cellular activities and to establish cell polarity.